NOS2-CD74 complex [GO:0035693] (cellular component) Relationships: is a type of protein-containing complex [GO:0032991] References: PMID:18003616 Sources: GOC:BHF Definition: A protein complex comprising nitric oxide synthase 2 and CD74. This stable complex formation is thought to prevent CD74 degradation by caspases.